negative regulation of reverse cholesterol transport [GO:1903063] (biological process) Relationships: is a type of negative regulation of cholesterol transport [GO:0032375]; is a type of regulation of reverse cholesterol transport [GO:1903062]; negatively regulates reverse cholesterol transport [GO:0043691] Definition: Any process that stops, prevents or reduces the frequency, rate or extent of reverse cholesterol transport. Also known as: down regulation of reverse cholesterol transport, down-regulation of reverse cholesterol transport, downregulation of reverse cholesterol transport, inhibition of reverse cholesterol transport References: PMID:23931754 Sources: GOC:BHF, GOC:TermGenie, GOC:rl, GO_REF:0000058